{
  "term_label": "detection of chemical stimulus involved in sensory perception of smell",
  "gene": "UniProtKB:Q8NG80",
  "gene_name": "Olfactory receptor 2L5",
  "term_id": "GO:0050911",
  "gene_symbol": "OR2L5"
}